{
  "gene": "UniProtKB:Q8NCM2",
  "gene_name": "Potassium voltage-gated channel subfamily H member 5",
  "term_id": "GO:0008076",
  "term_label": "voltage-gated potassium channel complex",
  "gene_symbol": "KCNH5"
}